{
  "term_id": "GO:0071880",
  "term_label": "adenylate cyclase-activating adrenergic receptor signaling pathway",
  "gene_name": "D(1B) dopamine receptor",
  "gene_symbol": "DRD5",
  "gene": "UniProtKB:P21918"
}